{
  "term_id": "GO:0045296",
  "gene": "UniProtKB:P19022",
  "gene_name": "Cadherin-2",
  "gene_symbol": "CDH2",
  "term_label": "cadherin binding"
}